{
  "term_id": "GO:0004435",
  "gene_symbol": "PLCB3",
  "term_label": "phosphatidylinositol-4,5-bisphosphate phospholipase C activity",
  "gene": "UniProtKB:Q01970",
  "gene_name": "1-phosphatidylinositol 4,5-bisphosphate phosphodiesterase beta-3"
}